{
  "gene_symbol": "IGHG3",
  "term_label": "antigen binding",
  "gene_name": "Immunoglobulin heavy constant gamma 3",
  "gene": "UniProtKB:P01860",
  "term_id": "GO:0003823"
}